{
  "gene_symbol": "CDK5R1",
  "term_label": "cyclin-dependent protein serine/threonine kinase activator activity",
  "gene": "UniProtKB:Q15078",
  "term_id": "GO:0061575",
  "gene_name": "Cyclin-dependent kinase 5 activator 1"
}